{
  "gene": "UniProtKB:Q7LBR1",
  "gene_symbol": "CHMP1B",
  "gene_name": "Charged multivesicular body protein 1b",
  "term_id": "GO:0015031",
  "term_label": "protein transport"
}